{
  "term_id": "GO:0005886",
  "gene_name": "Ras-related protein Rab-42",
  "term_label": "plasma membrane",
  "gene_symbol": "RAB42",
  "gene": "UniProtKB:Q8N4Z0"
}